cyclin E1-CDK2 complex [GO:0097134] (cellular component) Definition: A protein complex consisting of cyclin E1 and cyclin-dependent kinase 2 (CDK2). Cyclins are characterized by periodicity in protein abundance throughout the cell cycle. Cyclin-dependent kinases represent a family of serine/threonine protein kinases that become active upon binding to a cyclin regulatory partner. References: PMID:15935619 Sources: GOC:so Relationships: is a type of GO:0000307